{
  "gene": "UniProtKB:O75901",
  "gene_symbol": "RASSF9",
  "gene_name": "Ras association domain-containing protein 9",
  "term_label": "recycling endosome",
  "term_id": "GO:0055037"
}